cellodextrin catabolic process [GO:2000890] (biological process) Also known as: cellodextrin catabolism Relationships: is a type of oligosaccharide catabolic process [GO:0009313]; is a type of GO:1901027; is a type of cellodextrin metabolic process [GO:2000889] Sources: GOC:mengo_curators Definition: The chemical reactions and pathways resulting in the breakdown of a cellodextrin. Regulation: regulated by GO:2000927; negatively regulated by negative regulation of cellodextrin catabolic process [GO:2000928]; positively regulated by positive regulation of cellodextrin catabolic process [GO:2000929]